lipoprotein metabolic process [GO:0042157] (biological process) Definition: The chemical reactions and pathways involving any conjugated, water-soluble protein in which the covalently attached nonprotein group consists of a lipid or lipids. Sources: ISBN:0198506732 Also known as: lipoprotein metabolism Relationships: is_a protein metabolic process [GO:0019538] Subtypes: GO:0042158, lipoprotein catabolic process [GO:0042159], lipoprotein modification [GO:0042160] Regulation: regulated by regulation of lipoprotein metabolic process [GO:0050746]; RO_0002213 by positive regulation of lipoprotein metabolic process [GO:0050747]; negatively regulated by negative regulation of lipoprotein metabolic process [GO:0050748]